{
  "gene_symbol": "AGFG1",
  "gene": "UniProtKB:P52594",
  "term_id": "UNKNOWN:0001",
  "gene_name": "Arf-GAP domain and FG repeat-containing protein 1",
  "term_label": "Unknown molecular function"
}